CAAX-box protein processing [GO:0071586] (biological process) Definition: The second process in a series of specific posttranslational modifications to the CAAX box region of CAAX box proteins, in which the last three amino acids of the protein (AAX) are removed by proteolysis. Sources: GOC:mah Relationships: is a type of GO:0016485; is part of CAAX-box protein maturation [GO:0080120]